mitotic recombination-dependent replication fork processing [GO:1990426] (biological process) Also known as: homologous recombination-dependent replication fork processing, mitotic recombination involved in collapsed replication fork processing, mitotic recombination involved in recovery from replication fork arrest, mitotic recombination involved in recovery from replication fork stalling, homologous recombination dependent replication fork recovery, mitotic recombination involved in replication fork processing, mitotic recombination involved in replication fork restart, mitotic recombination involved in replication restart Definition: Replication fork processing that includes recombination between DNA near the arrested fork and homologous sequences. Proteins involved in homologous recombination are required for replication restart. Regulation: negatively regulated by GO:0120291; positively regulated by positive regulation of mitotic recombination-dependent replication fork processing [GO:0120292]; regulated by regulation of mitotic recombination-dependent replication fork processing [GO:1903221] References: PMID:23093942 Sources: GOC:mah Relationships: is a type of replication fork processing [GO:0031297]; is_a mitotic DNA replication maintenance of fidelity [GO:1990505]; has part mitotic recombination [GO:0006312]